oxytetracycline catabolic process [GO:1901762] (BP) Definition: The chemical reactions and pathways resulting in the breakdown of oxytetracycline. References: PMID:8163168 Sources: GOC:TermGenie, GOC:yaf Also known as: oxytetracycline breakdown, oxytetracycline catabolism, oxytetracycline degradation Relationships: is a type of GO:0030640